{
  "term_label": "cytoplasm",
  "term_id": "GO:0005737",
  "gene_name": "E3 ubiquitin-protein ligase HACE1",
  "gene": "UniProtKB:Q8IYU2",
  "gene_symbol": "HACE1"
}